{
  "gene_name": "Mucosa-associated lymphoid tissue lymphoma translocation protein 1",
  "gene": "UniProtKB:Q9UDY8",
  "term_label": "B cell activation",
  "term_id": "GO:0042113",
  "gene_symbol": "MALT1"
}